{
  "gene_name": "Zinc finger protein GLIS3",
  "gene_symbol": "GLIS3",
  "term_id": "GO:0005634",
  "term_label": "nucleus",
  "gene": "UniProtKB:Q8NEA6"
}